{
  "term_label": "eye development",
  "gene_name": "Homeobox protein Meis2",
  "term_id": "GO:0001654",
  "gene_symbol": "MEIS2",
  "gene": "UniProtKB:O14770"
}